{
  "gene": "UniProtKB:Q8WZ59",
  "gene_symbol": "TMEM190",
  "term_id": "GO:0002244",
  "gene_name": "Transmembrane protein 190",
  "term_label": "hematopoietic progenitor cell differentiation"
}